{
  "term_id": "GO:0005525",
  "term_label": "GTP binding",
  "gene_name": "Ras-related GTP-binding protein D",
  "gene_symbol": "RRAGD",
  "gene": "UniProtKB:Q9NQL2"
}